{
  "gene_name": "Coiled-coil domain-containing protein 149",
  "term_id": "UNKNOWN:0002",
  "gene": "UniProtKB:Q6ZUS6",
  "term_label": "Unknown biological process",
  "gene_symbol": "CCDC149"
}